maleylacetate reductase activity [GO:0018506] (molecular function) Definition: Catalysis of the reaction: 3-oxoadipate + NAD(P)+ = 2-maleylacetate + NAD(P)H + H+. Relationships: is a type of GO:0016628 Also known as: 3-oxoadipate:NAD(P)+ oxidoreductase activity, maleolylacetate reductase activity Sources: EC:1.3.1.32